detection of reduced oxygen by carotid body chemoreceptor signaling [GO:0003039] (biological process) Sources: GOC:mtg_cardio Relationships: is a type of detection of reduced oxygen by chemoreceptor signaling [GO:0003020]; BFO_0000050 detection of hypoxic conditions in blood by carotid body chemoreceptor signaling [GO:0003029] Definition: The process in which information about the levels of oxygen are received and are converted to a molecular signal by chemoreceptors in a carotid body. Also known as: detection of reduced oxygen by carotid body chemoreceptor signalling